{
  "term_label": "chromatin binding",
  "gene_name": "Nucleosome assembly protein 1-like 4",
  "gene_symbol": "NAP1L4",
  "term_id": "GO:0003682",
  "gene": "UniProtKB:Q99733"
}